{
  "term_id": "GO:0006635",
  "gene_symbol": "AUH",
  "gene": "UniProtKB:Q13825",
  "gene_name": "Methylglutaconyl-CoA hydratase, mitochondrial",
  "term_label": "fatty acid beta-oxidation"
}